{
  "term_id": "GO:0000978",
  "gene_name": "Homeobox protein Meis1",
  "term_label": "RNA polymerase II cis-regulatory region sequence-specific DNA binding",
  "gene_symbol": "MEIS1",
  "gene": "UniProtKB:O00470"
}